chloride transmembrane transporter activity [GO:0015108] (molecular function) Sources: GOC:ai Definition: Enables the transfer of chloride ions from one side of a membrane to the other. Subtypes: GO:0005254, chloride:monoatomic cation symporter activity [GO:0015377], chloride:proton antiporter activity [GO:0062158], chloride:bicarbonate antiporter activity [GO:0140900], GO:0160044, oxalate:chloride antiporter activity [GO:0160046] Also known as: chloride ion transmembrane transporter activity, ATP-dependent chloride transmembrane transporter activity, ATPase-coupled chloride transmembrane transporter activity, chloride ABC transporter, chloride transporting ATPase activity, chloride-transporting ATPase activity Relationships: is a type of monoatomic anion transmembrane transporter activity [GO:0008509]; is part of GO:1902476